{
  "gene_symbol": "SLC36A2",
  "term_label": "glycine transmembrane transporter activity",
  "term_id": "GO:0015187",
  "gene_name": "Proton-coupled amino acid transporter 2",
  "gene": "UniProtKB:Q495M3"
}